{
  "term_id": "UNKNOWN:0001",
  "term_label": "Unknown molecular function",
  "gene_symbol": "FOXRED1",
  "gene_name": "FAD-dependent oxidoreductase domain-containing protein 1",
  "gene": "UniProtKB:Q96CU9"
}